{
  "term_label": "BRCA1-A complex",
  "gene": "UniProtKB:Q8N594",
  "gene_name": "MPN domain-containing protein",
  "term_id": "GO:0070531",
  "gene_symbol": "MPND"
}